SCF ubiquitin ligase complex [GO:0019005] (cellular component) Relationships: is a type of GO:0031461 Subtypes: cytoplasmic SCF ubiquitin ligase complex [GO:0043223], nuclear SCF ubiquitin ligase complex [GO:0043224], SCF-Cdc4 ubiquitin ligase complex [GO:0097660], SCF-Ctf13 ubiquitin ligase complex [GO:0097661], SCF-Das1 ubiquitin ligase complex [GO:0097662], SCF-Dia2/Pof3 ubiquitin ligase complex [GO:0097663], SCF-Grr1/Pof2 ubiquitin ligase complex [GO:0097664], SCF-Mdm30 ubiquitin ligase complex [GO:0097665], SCF-Met30/Pof1 ubiquitin ligase complex [GO:0097666], GO:0097667, GO:0097668, GO:0097669, SCF-Ufo1/Pof10 ubiquitin ligase complex [GO:0097670], SCF-YDR131C ubiquitin ligase complex [GO:0097671], SCF-Pof5 ubiquitin ligase complex [GO:0097672], GO:0097673, GO:0097674, SCF-Hrt3/Pof7 ubiquitin ligase complex [GO:0097675] References: PMID:15571813, PMID:15688063 Also known as: CDL1 complex, CRL1 complex, Cul1-RING ubiquitin ligase complex, SCF complex, Skp1/Cul1/F-box protein complex, cullin-RING ligase 1, SCF complex substrate recognition subunit Definition: A ubiquitin ligase complex in which a cullin from the Cul1 subfamily and a RING domain protein form the catalytic core; substrate specificity is conferred by a Skp1 adaptor and an F-box protein. SCF complexes are involved in targeting proteins for degradation by the proteasome. The best characterized complexes are those from yeast and mammals (with core subunits named Cdc53/Cul1, Rbx1/Hrt1/Roc1).